{
  "gene_name": "Ubiquitin carboxyl-terminal hydrolase isozyme L5",
  "gene_symbol": "UCHL5",
  "term_label": "cytoplasm",
  "term_id": "GO:0005737",
  "gene": "UniProtKB:Q9Y5K5"
}